{
  "term_id": "UNKNOWN:0003",
  "gene_name": "NPC intracellular cholesterol transporter 2",
  "gene": "UniProtKB:P61916",
  "term_label": "Unknown cellular component",
  "gene_symbol": "NPC2"
}